{
  "gene_name": "Spectrin beta chain, erythrocytic",
  "term_id": "GO:0030036",
  "term_label": "actin cytoskeleton organization",
  "gene_symbol": "SPTB",
  "gene": "UniProtKB:P11277"
}